{
  "term_label": "Unknown molecular function",
  "term_id": "UNKNOWN:0001",
  "gene_name": "Squamous cell carcinoma antigen recognized by T-cells 3",
  "gene": "UniProtKB:Q15020",
  "gene_symbol": "SART3"
}